{
  "gene": "UniProtKB:Q6ZP65",
  "term_id": "UNKNOWN:0001",
  "gene_symbol": "BICDL1",
  "term_label": "Unknown molecular function",
  "gene_name": "BICD family-like cargo adapter 1"
}